{
  "gene": "UniProtKB:P62875",
  "term_id": "GO:0006366",
  "gene_symbol": "POLR2L",
  "gene_name": "DNA-directed RNA polymerases I, II, and III subunit RPABC5",
  "term_label": "transcription by RNA polymerase II"
}